intramolecular transferase activity [GO:0016866] (molecular function) Definition: Catalysis of the transfer of a functional group from one position to another within a single molecule. Subtypes: chorismate mutase activity [GO:0004106], methylmalonyl-CoA mutase activity [GO:0004494], GO:0008767, pseudouridine synthase activity [GO:0009982], intramolecular acyltransferase activity [GO:0016867], intramolecular phosphotransferase activity [GO:0016868], intramolecular aminotransferase activity [GO:0016869], oxidosqualene cyclase activity [GO:0031559], 5-(carboxyamino)imidazole ribonucleotide mutase activity [GO:0034023], pivalyl-CoA mutase activity [GO:0034784], GO:0047469, (1,4)-alpha-D-glucan 1-alpha-D-glucosylmutase activity [GO:0047470], maltose alpha-D-glucosyltransferase activity [GO:0047471], 2-acetolactate mutase activity [GO:0047534], 2-methyleneglutarate mutase activity [GO:0047548], isobutyryl-CoA mutase activity [GO:0047727], isomaltulose synthase activity [GO:0050006], GO:0050097, GO:0050486, squalene-hopene cyclase activity [GO:0051007], UDP-arabinopyranose mutase activity [GO:0052691], D-ribose pyranase activity [GO:0062193], camelliol C synthase activity [GO:0090438] Relationships: is a type of isomerase activity [GO:0016853] Sources: GOC:mah Also known as: mutase activity, intramolecular transferase activity, transferring other groups